{
  "term_label": "Unknown cellular component",
  "gene_symbol": "NEK1",
  "gene_name": "Serine_threonine-protein kinase Nek1",
  "gene": "UniProtKB:Q96PY6",
  "term_id": "UNKNOWN:0003"
}